glycerol-3-phosphate metabolic process [GO:0006072] (biological process) Relationships: is a type of alditol phosphate metabolic process [GO:0052646] Definition: The chemical reactions and pathways involving glycerol-3-phosphate, a phosphoric monoester of glycerol. Also known as: glycerol-3-phosphate metabolism Subtypes: glycerol-3-phosphate biosynthetic process [GO:0046167], glycerol-3-phosphate catabolic process [GO:0046168] Sources: GOC:go_curators, ISBN:0198506732